{
  "gene_symbol": "BPIFB3",
  "term_label": "Unknown cellular component",
  "term_id": "UNKNOWN:0003",
  "gene": "UniProtKB:P59826",
  "gene_name": "BPI fold-containing family B member 3"
}